cobalamin transport [GO:0015889] (biological process) Sources: GOC:ai Definition: The directed movement of cobalamin (vitamin B12), a water-soluble vitamin characterized by possession of a corrin nucleus containing a cobalt atom, into, out of or within a cell, or between cells, by means of some agent such as a transporter or pore. Also known as: vitamin B12 transport Relationships: is a type of GO:0051180; is a type of nitrogen compound transport [GO:0071705]